{
  "term_id": "UNKNOWN:0001",
  "gene_symbol": "TMEM176B",
  "gene": "UniProtKB:Q3YBM2",
  "term_label": "Unknown molecular function",
  "gene_name": "Transmembrane protein 176B"
}